regulation of neural crest cell differentiation [GO:1905292] (biological process) Definition: Any process that modulates the frequency, rate or extent of neural crest cell differentiation. Relationships: is a type of regulation of stem cell differentiation [GO:2000736]; regulates neural crest cell differentiation [GO:0014033] References: PMID:15073157 Sources: GOC:BHF, GOC:TermGenie, GOC:rl, GO_REF:0000058 Subtypes: negative regulation of neural crest cell differentiation [GO:1905293], GO:1905294, regulation of neural crest cell fate specification [GO:1905295]